{
  "gene": "UniProtKB:Q96J42",
  "term_id": "GO:0060271",
  "gene_symbol": "TXNDC15",
  "term_label": "cilium assembly",
  "gene_name": "Thioredoxin domain-containing protein 15"
}